estrogen catabolic process [GO:0006711] (biological process) Definition: The chemical reactions and pathways resulting in the breakdown of estrogens, C18 steroid hormones that can stimulate the development of female sexual characteristics. Also found in plants. Sources: ISBN:0198506732 Also known as: estrogen breakdown, estrogen catabolism, estrogen degradation, oestrogen catabolic process, oestrogen catabolism Relationships: is a type of steroid catabolic process [GO:0006706]; is a type of GO:0008210; is a type of hormone catabolic process [GO:0042447]